{
  "gene_symbol": "RNF139",
  "term_label": "endomembrane system",
  "gene_name": "E3 ubiquitin-protein ligase RNF139",
  "term_id": "GO:0012505",
  "gene": "UniProtKB:Q8WU17"
}